{
  "term_label": "sperm flagellum",
  "gene_symbol": "CFAP251",
  "gene_name": "Cilia- and flagella-associated protein 251",
  "term_id": "GO:0036126",
  "gene": "UniProtKB:Q8TBY9"
}